{
  "gene": "UniProtKB:Q96JQ5",
  "term_id": "UNKNOWN:0002",
  "gene_name": "Membrane-spanning 4-domains subfamily A member 4A",
  "gene_symbol": "MS4A4A",
  "term_label": "Unknown biological process"
}